retinal rod cell development [GO:0046548] (biological process) Relationships: is a type of GO:0042462; is part of retinal rod cell differentiation [GO:0060221] Sources: ISBN:0198506732 Definition: Development of a rod cell, one of the sensory cells in the eye that reacts to the presence of light. Rod cells contain the photopigment rhodopsin or porphyropsin and are responsible for vision in dim light.